{
  "term_label": "positive regulation of lipopolysaccharide-mediated signaling pathway",
  "gene_name": "CD180 antigen",
  "gene": "UniProtKB:Q99467",
  "term_id": "GO:0031666",
  "gene_symbol": "CD180"
}